{
  "term_id": "GO:0005634",
  "gene_name": "T-box transcription factor TBX5",
  "gene": "UniProtKB:Q99593",
  "gene_symbol": "TBX5",
  "term_label": "nucleus"
}